negative regulation of lysine biosynthetic process via aminoadipic acid [GO:1902987] (biological process) Definition: Any process that stops, prevents or reduces the frequency, rate or extent of lysine biosynthetic process via aminoadipic acid. Relationships: is a type of negative regulation of small molecule metabolic process [GO:0062014]; is a type of regulation of lysine biosynthetic process via aminoadipic acid [GO:1902986]; is a type of negative regulation of amino acid biosynthetic process [GO:2000283]; negatively regulates GO:0019878 References: PMID:8590464 Sources: GOC:TermGenie, GO_REF:0000058 Subtypes: negative regulation of lysine biosynthetic process via alpha-aminoadipate and saccharopine [GO:2001195] Also known as: down regulation of lysine anabolism via aminoadipic acid, down regulation of lysine biosynthesis, aminoadipic acid pathway, down regulation of lysine biosynthesis, aminoadipic pathway, down regulation of lysine biosynthetic process via aminoadipic acid, down regulation of lysine biosynthetic process, aminoadipic acid pathway, down regulation of lysine biosynthetic process, aminoadipic pathway, down regulation of lysine formation via aminoadipic acid, down regulation of lysine synthesis via aminoadipic acid, down-regulation of lysine anabolism via aminoadipic acid, down-regulation of lysine biosynthesis, aminoadipic acid pathway, down-regulation of lysine biosynthesis, aminoadipic pathway, down-regulation of lysine biosynthetic process via aminoadipic acid, down-regulation of lysine biosynthetic process, aminoadipic acid pathway, down-regulation of lysine biosynthetic process, aminoadipic pathway, down-regulation of lysine formation via aminoadipic acid, down-regulation of lysine synthesis via aminoadipic acid, downregulation of lysine anabolism via aminoadipic acid, downregulation of lysine biosynthesis, aminoadipic acid pathway, downregulation of lysine biosynthesis, aminoadipic pathway, downregulation of lysine biosynthetic process via aminoadipic acid, downregulation of lysine biosynthetic process, aminoadipic acid pathway, downregulation of lysine biosynthetic process, aminoadipic pathway, downregulation of lysine formation via aminoadipic acid, downregulation of lysine synthesis via aminoadipic acid, negative regulation of lysine anabolism via aminoadipic acid, negative regulation of lysine biosynthesis, aminoadipic acid pathway, negative regulation of lysine biosynthesis, aminoadipic pathway, negative regulation of lysine biosynthetic process, aminoadipic acid pathway, negative regulation of lysine biosynthetic process, aminoadipic pathway, negative regulation of lysine formation via aminoadipic acid, negative regulation of lysine synthesis via aminoadipic acid, inhibition of lysine anabolism via aminoadipic acid, inhibition of lysine biosynthesis, aminoadipic acid pathway, inhibition of lysine biosynthesis, aminoadipic pathway, inhibition of lysine biosynthetic process via aminoadipic acid, inhibition of lysine biosynthetic process, aminoadipic acid pathway, inhibition of lysine biosynthetic process, aminoadipic pathway, inhibition of lysine formation via aminoadipic acid, inhibition of lysine synthesis via aminoadipic acid